{
  "term_label": "Unknown biological process",
  "gene_symbol": "C5orf24",
  "gene_name": "UPF0461 protein C5orf24",
  "term_id": "UNKNOWN:0002",
  "gene": "UniProtKB:Q7Z6I8"
}